wing disc proximal/distal pattern formation [GO:0007473] (biological process) Relationships: is a type of proximal/distal pattern formation, imaginal disc [GO:0007449]; is a type of wing disc pattern formation [GO:0035222] Sources: GOC:bf Definition: The establishment, maintenance and elaboration of the proximal/distal axis of the wing disc, a precursor to the adult wing.